negative regulation of cell cycle switching, mitotic to meiotic cell cycle [GO:0110045] (biological process) Definition: Any process that stops, prevents, or reduces the frequency, rate, or extent of mitotic to meiotic cell cycle switching, the process in which a cell switches cell cycle mode from mitotic to meiotic division. References: PMID:17674143 Sources: GOC:al Relationships: is a type of GO:0010948; is a type of positive regulation of mitotic cell cycle [GO:0045931]; is a type of regulation of cell cycle switching, mitotic to meiotic cell cycle [GO:0110044]; negatively regulates cell cycle switching, mitotic to meiotic cell cycle [GO:0051728]